{
  "gene_name": "Putative histone H2B type 2-D",
  "term_label": "extracellular space",
  "gene_symbol": "H2BC19P",
  "term_id": "GO:0005615",
  "gene": "UniProtKB:Q6DRA6"
}